{
  "term_label": "hyaluronan biosynthetic process",
  "gene_symbol": "HAS2",
  "gene": "UniProtKB:Q92819",
  "term_id": "GO:0030213",
  "gene_name": "Hyaluronan synthase 2"
}